{
  "term_label": "transcription factor TFIID complex",
  "term_id": "GO:0005669",
  "gene_symbol": "TAF13",
  "gene_name": "Transcription initiation factor TFIID subunit 13",
  "gene": "UniProtKB:Q15543"
}